{
  "term_id": "GO:0005634",
  "term_label": "nucleus",
  "gene_symbol": "ZNF473",
  "gene": "UniProtKB:Q8WTR7",
  "gene_name": "Zinc finger protein 473"
}